{
  "term_id": "UNKNOWN:0001",
  "term_label": "Unknown molecular function",
  "gene_name": "Ankyrin repeat domain-containing protein 20B",
  "gene_symbol": "ANKRD20A8P",
  "gene": "UniProtKB:Q5CZ79"
}